{
  "gene": "UniProtKB:P23945",
  "term_label": "hormone-mediated signaling pathway",
  "gene_symbol": "FSHR",
  "gene_name": "Follicle-stimulating hormone receptor",
  "term_id": "GO:0009755"
}